{
  "gene_name": "Intermediate conductance calcium-activated potassium channel protein 4",
  "term_id": "GO:0071805",
  "gene_symbol": "KCNN4",
  "gene": "UniProtKB:O15554",
  "term_label": "potassium ion transmembrane transport"
}